{
  "term_id": "GO:0005886",
  "gene_name": "Metalloreductase STEAP4",
  "term_label": "plasma membrane",
  "gene": "UniProtKB:Q687X5",
  "gene_symbol": "STEAP4"
}